{
  "term_id": "GO:0045071",
  "gene_name": "2-5A-dependent ribonuclease",
  "term_label": "negative regulation of viral genome replication",
  "gene": "UniProtKB:Q05823",
  "gene_symbol": "RNASEL"
}